embryonic crystal cell differentiation [GO:0035165] (biological process) Relationships: is a type of GO:0035163; is a type of crystal cell differentiation [GO:0042688] Definition: The process in which an embryonic mesoderm-derived hemocyte precursor cell acquires the specialized features of a crystal cell. Crystal cells are a class of cells that contain crystalline inclusions and are involved in the melanization of pathogenic material in the hemolymph. Sources: GOC:bf, http://sdb.bio.purdue.edu/fly/gene/serpent3.htm